{
  "gene_symbol": "MUL1",
  "term_label": "ubiquitin protein ligase activity",
  "gene": "UniProtKB:Q969V5",
  "gene_name": "Mitochondrial ubiquitin ligase activator of NFKB 1",
  "term_id": "GO:0061630"
}